{
  "gene": "UniProtKB:Q8NAU1",
  "gene_name": "Fibronectin type III domain-containing protein 5",
  "gene_symbol": "FNDC5",
  "term_label": "Unknown molecular function",
  "term_id": "UNKNOWN:0001"
}